{
  "term_id": "GO:0030054",
  "gene_name": "Epiplakin",
  "gene_symbol": "EPPK1",
  "term_label": "cell junction",
  "gene": "UniProtKB:P58107"
}